short-day photoperiodism, flowering [GO:0048575] (biological process) Definition: A change from vegetative to reproductive phase as a result of detection of, or exposure to, a period of light that falls short of the critical day length. The critical day length varies between species. Although the term is short-day is used, most species actually respond to the duration of the night, so that the response will occur when a period of darkness exceeds the number of hours defined by 24 minus the critical day length. Sources: GOC:jid, GOC:pj, ISBN:0582015952, ISBN:0697037754, ISBN:0709408862 Regulation: positively regulated by GO:0048576; negatively regulated by negative regulation of short-day photoperiodism, flowering [GO:0048577]; regulated by regulation of short-day photoperiodism, flowering [GO:0048587] Also known as: long-night photoperiodism, flowering, response to long-night, flowering, response to short-day, flowering, short-day photoperiodic control of flowering, short-day photoperiodic control of flowering time, short-day photoperiodic control of inflorescence development Relationships: is a type of short-day photoperiodism [GO:0048572]; is a type of photoperiodism, flowering [GO:0048573]